{
  "gene_name": "Serpin A12",
  "gene": "UniProtKB:Q8IW75",
  "term_id": "GO:0004867",
  "term_label": "serine-type endopeptidase inhibitor activity",
  "gene_symbol": "SERPINA12"
}